positive regulation of execution phase of apoptosis [GO:1900119] (biological process) Relationships: is a type of positive regulation of apoptotic process [GO:0043065]; is a type of regulation of execution phase of apoptosis [GO:1900117]; positively regulates execution phase of apoptosis [GO:0097194] Sources: GOC:TermGenie, GOC:mtg_apoptosis Definition: Any process that activates or increases the frequency, rate or extent of execution phase of apoptosis. Also known as: up regulation of execution phase of apoptosis, up-regulation of execution phase of apoptosis, upregulation of execution phase of apoptosis, activation of execution phase of apoptosis